gamma-aminobutyric acid biosynthetic process [GO:0009449] (biological process) Note: See also the biological process term 'neurotransmitter biosynthetic process ; GO:0042136'. Relationships: is a type of amino acid biosynthetic process [GO:0008652]; is a type of GO:0009448; is a type of GO:0170043 Sources: GOC:ai Definition: The chemical reactions and pathways resulting in the formation of gamma-aminobutyric acid (GABA, 4-aminobutyrate), an amino acid which acts as a neurotransmitter in some organisms. Also known as: 4-aminobutanoate biosynthesis, 4-aminobutanoate biosynthetic process, 4-aminobutyrate biosynthesis, 4-aminobutyrate biosynthetic process, GABA biosynthesis, GABA biosynthetic process, gamma-aminobutyric acid anabolism, gamma-aminobutyric acid biosynthesis, gamma-aminobutyric acid formation, gamma-aminobutyric acid synthesis